{
  "gene_symbol": "MMD",
  "term_id": "UNKNOWN:0002",
  "term_label": "Unknown biological process",
  "gene_name": "Monocyte to macrophage differentiation factor",
  "gene": "UniProtKB:Q15546"
}